{
  "term_label": "Golgi apparatus",
  "term_id": "GO:0005794",
  "gene_symbol": "ARV1",
  "gene_name": "Protein ARV1",
  "gene": "UniProtKB:Q9H2C2"
}